negative regulation of palmitic acid catabolic process [GO:0106394] (biological process) Definition: Any process that stops, prevents or reduces the frequency, rate or extent of a palmitic acid catabolic process. References: PMID:14677856 Relationships: is a type of negative regulation of fatty acid metabolic process [GO:0045922]; is a type of GO:0050995; is a type of regulation of palmitic acid catabolic process [GO:0106393]; negatively regulates palmitic acid catabolic process [GO:1900534]